phosphopantothenate--cysteine ligase activity [GO:0004632] (molecular function) Also known as: phosphopantothenate-cysteine ligase activity, phosphopantothenoylcysteine synthetase activity, (R)-4'-phosphopantothenate:L-cysteine ligase activity Sources: EC:6.3.2.5 Definition: Catalysis of the reaction: CTP + (R)-4'-phosphopantothenate + L-cysteine = CMP + diphosphate + (R)-4'-phosphopantothenoyl-L-cysteine. Cysteine can be replaced by some of its derivatives. Relationships: is a type of acid-amino acid ligase activity [GO:0016881]